dermatan 2-sulfotransferase activity [GO:0102142] (molecular function) Definition: Catalysis of the reaction: dermatan-[core protein] + 3'-phosphoadenylyl-sulfate = [dermatan-sulfate] containing 2-O-sulfo-alpha-L-iduronate + adenosine 3',5'-bisphosphate + H+. Sources: MetaCyc:RXN-11561 Relationships: is a type of dermatan sulfotransferase activity [GO:0120534] Also known as: [dermatan sulfate]-L-iduronyl 2-Osulfotransferase activity